{
  "gene": "UniProtKB:Q6ZT62",
  "gene_symbol": "BARGIN",
  "term_label": "GTPase activator activity",
  "term_id": "GO:0005096",
  "gene_name": "Bargin"
}